negative regulation of nucleobase-containing compound transport [GO:0032240] (biological process) Definition: Any process that stops, prevents, or reduces the frequency, rate or extent of the directed movement of nucleobases, nucleosides, nucleotides and nucleic acids, into, out of or within a cell, or between cells, by means of some agent such as a transporter or pore. Sources: GOC:mah Also known as: down regulation of nucleobase, nucleoside, nucleotide and nucleic acid transport, down-regulation of nucleobase, nucleoside, nucleotide and nucleic acid transport, downregulation of nucleobase, nucleoside, nucleotide and nucleic acid transport, inhibition of nucleobase, nucleoside, nucleotide and nucleic acid transport, negative regulation of nucleobase, nucleoside, nucleotide and nucleic acid transport Relationships: is a type of regulation of nucleobase-containing compound transport [GO:0032239]; is a type of negative regulation of transport [GO:0051051]; negatively regulates nucleobase-containing compound transport [GO:0015931] Subtypes: negative regulation of nucleoside transport [GO:0032243], negative regulation of hypoxanthine transport [GO:0035347], negative regulation of thymine transport [GO:0035366], negative regulation of RNA import into nucleus [GO:0046829], negative regulation of RNA export from nucleus [GO:0046832]